{
  "term_label": "plasma membrane",
  "gene": "UniProtKB:Q7RTX1",
  "term_id": "GO:0005886",
  "gene_symbol": "TAS1R1",
  "gene_name": "Taste receptor type 1 member 1"
}